{
  "gene_symbol": "IL16",
  "term_id": "GO:0005125",
  "gene": "UniProtKB:Q14005",
  "term_label": "cytokine activity",
  "gene_name": "Pro-interleukin-16"
}